{
  "term_label": "Unknown molecular function",
  "term_id": "UNKNOWN:0001",
  "gene_symbol": "SPATA1",
  "gene_name": "Spermatogenesis-associated protein 1",
  "gene": "UniProtKB:Q5VX52"
}